thiol sulfotransferase activity [GO:0033870] (molecular function) Also known as: PAPS sulfotransferase activity, 3'-phosphoadenylyl-sulfate:thiol S-sulfotransferase activity, adenosine 3'-phosphate 5'-sulphatophosphate sulfotransferase activity Sources: EC:2.8.2.16 Definition: Catalysis of the reaction: 3'-phosphoadenylyl sulfate + a thiol = adenosine 3',5'-bisphosphate + an S-alkyl thiosulfate. Relationships: is a type of sulfotransferase activity [GO:0008146]